{
  "term_id": "GO:0006633",
  "gene_symbol": "FASN",
  "gene": "UniProtKB:P49327",
  "term_label": "fatty acid biosynthetic process",
  "gene_name": "Fatty acid synthase"
}